{
  "gene_symbol": "KCNE3",
  "term_id": "GO:0086011",
  "gene_name": "Potassium voltage-gated channel subfamily E member 3",
  "gene": "UniProtKB:Q9Y6H6",
  "term_label": "membrane repolarization during action potential"
}